{
  "gene_symbol": "NACC1",
  "term_label": "DNA-binding transcription factor activity, RNA polymerase II-specific",
  "gene_name": "Nucleus accumbens-associated protein 1",
  "gene": "UniProtKB:Q96RE7",
  "term_id": "GO:0000981"
}